{
  "gene_name": "Transcription factor SOX-14",
  "term_id": "GO:0000978",
  "gene": "UniProtKB:O95416",
  "term_label": "RNA polymerase II cis-regulatory region sequence-specific DNA binding",
  "gene_symbol": "SOX14"
}